trochlear nerve structural organization [GO:0021641] (biological process) Also known as: trochlear nerve structural organisation, CN IV structural organization Sources: GOC:cls, GOC:dgh, GOC:dph, GOC:jid, GO_REF:0000021 Definition: The process that contributes to the act of creating the structural organization of the trochlear nerve. This process pertains to the physical shaping of a rudimentary structure. The trochlear nerve is a motor nerve and is the only cranial nerve to exit the brain dorsally. The trochlear nerve innervates the superior oblique muscle. Relationships: is a type of cranial nerve structural organization [GO:0021604]; is part of GO:0021639